ribosome biogenesis [GO:0042254] (biological process) References: PMID:26404467 Sources: GOC:ma, Wikipedia:Ribosome_biogenesis Definition: A cellular process that results in the biosynthesis of constituent macromolecules, assembly, and arrangement of constituent parts of ribosome subunits; includes transport to the sites of protein synthesis. Relationships: is a type of ribonucleoprotein complex biogenesis [GO:0022613] Regulation: regulated by regulation of ribosome biogenesis [GO:0090069]; positively regulated by positive regulation of ribosome biogenesis [GO:0090070]; negatively regulated by negative regulation of ribosome biogenesis [GO:0090071] Also known as: ribosome biogenesis and assembly